{
  "term_label": "extracellular space",
  "gene": "UniProtKB:O75596",
  "gene_name": "C-type lectin domain family 3 member A",
  "gene_symbol": "CLEC3A",
  "term_id": "GO:0005615"
}